{
  "term_label": "Unknown cellular component",
  "gene": "UniProtKB:Q8IYS8",
  "term_id": "UNKNOWN:0003",
  "gene_name": "Biorientation of chromosomes in cell division protein 1-like 2",
  "gene_symbol": "BOD1L2"
}